{
  "gene_symbol": "SMUG1",
  "gene_name": "Single-strand selective monofunctional uracil DNA glycosylase",
  "gene": "UniProtKB:Q53HV7",
  "term_id": "UNKNOWN:0003",
  "term_label": "Unknown cellular component"
}